{
  "gene": "UniProtKB:P29536",
  "term_label": "muscle contraction",
  "gene_symbol": "LMOD1",
  "term_id": "GO:0006936",
  "gene_name": "Leiomodin-1"
}